{
  "term_id": "GO:0008333",
  "term_label": "endosome to lysosome transport",
  "gene_name": "Pleckstrin homology domain-containing family F member 2",
  "gene_symbol": "PLEKHF2",
  "gene": "UniProtKB:Q9H8W4"
}